medullary reticular formation development [GO:0021723] (biological process) Sources: GOC:cjm, GOC:cls, GOC:curators, GOC:dgh, GOC:dph Definition: The process whose specific outcome is the progression of the medullary reticular formation over time, from its formation to the mature structure. The medullary reticular formation is a series of brain nuclei located in the medulla oblongata. Relationships: is_a GO:0048856; is part of medulla oblongata development [GO:0021550] Also known as: rhombencephalic reticular formation development